positive regulation of protein-containing complex disassembly [GO:0043243] (biological process) Sources: GOC:jl Relationships: is a type of regulation of protein-containing complex disassembly [GO:0043244]; is a type of positive regulation of cellular component organization [GO:0051130]; positively regulates protein-containing complex disassembly [GO:0032984] Definition: Any process that activates or increases the frequency, rate or extent of protein complex disassembly, the disaggregation of a protein complex into its constituent components. Subtypes: GO:0035540, positive regulation of translational termination [GO:0045905], GO:0060566, GO:1901098, GO:1901881 Also known as: up regulation of protein complex disassembly, up-regulation of protein complex disassembly, upregulation of protein complex disassembly, activation of protein complex disassembly, stimulation of protein complex disassembly, positive regulation of protein complex disassembly